{
  "gene_symbol": "MOGAT3",
  "term_id": "GO:0019432",
  "gene": "UniProtKB:Q86VF5",
  "term_label": "triglyceride biosynthetic process",
  "gene_name": "2-acylglycerol O-acyltransferase 3"
}